{
  "gene": "UniProtKB:Q15669",
  "gene_symbol": "RHOH",
  "term_id": "GO:0007165",
  "gene_name": "Rho-related GTP-binding protein RhoH",
  "term_label": "signal transduction"
}